indoleacetic acid ester conjugate biosynthetic process [GO:0033476] (biological process) Sources: GOC:mah, MetaCyc:PWY-1741 Definition: The chemical reactions and pathways resulting in the formation of an indole-3-acetic acid amide conjugate, a form of indoleacetic acid covalently bound to an a sugar or polyol through an ester bond. Also known as: IAA ester conjugate biosynthetic process, indole acetic acid ester conjugate biosynthesis, indole acetic acid ester conjugate biosynthetic process, indoleacetic acid ester conjugate anabolism, indoleacetic acid ester conjugate biosynthesis, indoleacetic acid ester conjugate formation, indoleacetic acid ester conjugate synthesis Relationships: is_a indoleacetic acid conjugate biosynthetic process [GO:0033474]